glycine import across plasma membrane [GO:1903804] (biological process) Definition: The directed movement of glycine from outside of a cell, across the plasma membrane and into the cytosol. References: PMID:23895341 Sources: GOC:TermGenie, GO_REF:0000075 Also known as: glycine import, glycine import into cell Relationships: is a type of glycine transport [GO:0015816]; is a type of amino acid import across plasma membrane [GO:0089718]; is a type of GO:1905039 Regulation: RO_0002211 by regulation of glycine import across plasma membrane [GO:1900923]; RO_0002212 by GO:1900924; RO_0002213 by positive regulation of glycine import across plasma membrane [GO:1900925]